{
  "term_id": "GO:0005737",
  "gene_symbol": "MKNK1",
  "term_label": "cytoplasm",
  "gene": "UniProtKB:Q9BUB5",
  "gene_name": "MAP kinase-interacting serine_threonine-protein kinase 1"
}